positive regulation of guanylate cyclase activity [GO:0031284] (BP) Definition: Any process that activates or increases the frequency, rate or extent of guanylate cyclase activity. Sources: GOC:mah Also known as: up regulation of guanylate cyclase activity, up-regulation of guanylate cyclase activity, upregulation of guanylate cyclase activity, activation of guanylate cyclase activity, stimulation of guanylate cyclase activity Relationships: is_a positive regulation of cyclase activity [GO:0031281]; is a type of positive regulation of lyase activity [GO:0051349]; is a type of positive regulation of purine nucleotide biosynthetic process [GO:1900373]; positively regulates guanylate cyclase activity [GO:0004383]